negative regulation of ascus development [GO:0075320] (BP) Sources: GOC:pamgo_curators Relationships: is a type of negative regulation of spore-bearing organ development [GO:0075262]; is a type of regulation of ascus development [GO:0075318]; negatively regulates ascus development [GO:0075317] Definition: Any process that stops, prevents, or reduces the frequency, rate or extent of ascus development, a saclike structure produced by fungi of the phylum Ascomycota (sac fungi) in which sexually produced spores (ascospores), usually four or eight in number, are formed.